digestive tract mesoderm development [GO:0007502] (biological process) Sources: GOC:ai Definition: The process whose specific outcome is the progression of the digestive tract mesoderm over time, from its formation to the mature structure. The digestive tract mesoderm is portion of the middle layer of the three primary germ layers of the embryo which will go on to form part of the digestive tract of the organism. Relationships: is a type of tissue development [GO:0009888]; is part of mesoderm development [GO:0007498]; is part of digestive tract development [GO:0048565]